{
  "term_label": "Unknown molecular function",
  "gene_symbol": "TTTY10",
  "gene_name": "Putative transcript Y 10 protein",
  "term_id": "UNKNOWN:0001",
  "gene": "UniProtKB:Q9BZA0"
}